{
  "gene_name": "Paired box protein Pax-6",
  "term_id": "GO:0060041",
  "gene": "UniProtKB:P26367",
  "term_label": "retina development in camera-type eye",
  "gene_symbol": "PAX6"
}